{
  "term_id": "GO:0030488",
  "gene_symbol": "TYW3",
  "gene": "UniProtKB:Q6IPR3",
  "term_label": "tRNA methylation",
  "gene_name": "tRNA wybutosine-synthesizing protein 3 homolog"
}